osteoblast differentiation [GO:0001649] (biological process) Sources: CL:0000062, GOC:jid, GO_REF:0000034 Definition: The process whereby a relatively unspecialized cell acquires the specialized features of an osteoblast, a mesodermal or neural crest cell that gives rise to bone. Regulation: regulated by regulation of osteoblast differentiation [GO:0045667]; negatively regulated by negative regulation of osteoblast differentiation [GO:0045668]; positively regulated by positive regulation of osteoblast differentiation [GO:0045669] Relationships: is a type of cell differentiation [GO:0030154]; is part of ossification [GO:0001503] Also known as: osteoblast cell differentiation